{
  "term_label": "Unknown molecular function",
  "term_id": "UNKNOWN:0001",
  "gene_name": "Ras-like protein family member 11A",
  "gene": "UniProtKB:Q6T310",
  "gene_symbol": "RASL11A"
}